{
  "term_label": "response to endoplasmic reticulum stress",
  "gene_symbol": "ERP27",
  "gene_name": "Endoplasmic reticulum resident protein 27",
  "gene": "UniProtKB:Q96DN0",
  "term_id": "GO:0034976"
}